{
  "term_label": "histone reader activity",
  "term_id": "GO:0140566",
  "gene_name": "Bromodomain-containing protein 7",
  "gene": "UniProtKB:Q9NPI1",
  "gene_symbol": "BRD7"
}